{
  "term_id": "UNKNOWN:0003",
  "gene_name": "Carbohydrate sulfotransferase 8",
  "gene": "UniProtKB:Q9H2A9",
  "gene_symbol": "CHST8",
  "term_label": "Unknown cellular component"
}